lactaldehyde reductase (NADPH) activity [GO:0050039] (molecular function) Also known as: 1,2-propanediol:NADP+ oxidoreductase activity, NADP-1,2-propanediol dehydrogenase activity, lactaldehyde (reduced nicotinamide adenine dinucleotide phosphate) reductase activity, propane-1,2-diol:NADP+ oxidoreductase activity, propanediol dehydrogenase activity Definition: Catalysis of the reaction: NADP+ + propane-1,2-diol = (S)-lactaldehyde + H+ + NADPH. Relationships: is a type of oxidoreductase activity, acting on the CH-OH group of donors, NAD or NADP as acceptor [GO:0016616] Sources: RHEA:15885